{
  "gene_name": "Synaptic vesicle glycoprotein 2A",
  "gene": "UniProtKB:Q7L0J3",
  "gene_symbol": "SV2A",
  "term_id": "GO:0043005",
  "term_label": "neuron projection"
}